{
  "gene_symbol": "ZNF101",
  "term_label": "DNA-binding transcription factor activity, RNA polymerase II-specific",
  "gene_name": "Zinc finger protein 101",
  "term_id": "GO:0000981",
  "gene": "UniProtKB:Q8IZC7"
}